{
  "term_id": "GO:0009986",
  "gene_name": "Putative teratocarcinoma-derived growth factor 3",
  "term_label": "cell surface",
  "gene": "UniProtKB:P51864",
  "gene_symbol": "CRIPTO3"
}